{
  "gene": "UniProtKB:Q8N5S3",
  "term_label": "Unknown cellular component",
  "gene_symbol": "C2orf73",
  "gene_name": "Uncharacterized protein C2orf73",
  "term_id": "UNKNOWN:0003"
}